{
  "term_id": "UNKNOWN:0001",
  "gene_name": "Immunoglobulin superfamily member 8",
  "gene_symbol": "IGSF8",
  "gene": "UniProtKB:Q969P0",
  "term_label": "Unknown molecular function"
}